{
  "gene_symbol": "GALT",
  "gene": "UniProtKB:P07902",
  "gene_name": "Galactose-1-phosphate uridylyltransferase",
  "term_id": "GO:0008108",
  "term_label": "UDP-glucose:hexose-1-phosphate uridylyltransferase activity"
}